{
  "term_id": "UNKNOWN:0002",
  "gene": "UniProtKB:P0CG13",
  "gene_symbol": "CHTF8",
  "term_label": "Unknown biological process",
  "gene_name": "Chromosome transmission fidelity protein 8 homolog"
}